negative regulation of triglyceride metabolic process [GO:0090209] (biological process) Sources: GOC:dph, GOC:sl, GOC:tb Definition: Any process that decreases the frequency, rate or extent of the chemical reactions and pathways involving triglyceride, any triester of glycerol. Relationships: is a type of negative regulation of lipid metabolic process [GO:0045833]; is a type of regulation of triglyceride metabolic process [GO:0090207]; negatively regulates triglyceride metabolic process [GO:0006641] Subtypes: GO:0010868, negative regulation of triglyceride catabolic process [GO:0010897]